metanephric glomerular parietal epithelial cell fate commitment [GO:0072247] (BP) Relationships: is_a GO:0072147; is a type of metanephric glomerular epithelial cell fate commitment [GO:0072315]; is part of GO:0072245 Sources: GOC:mtg_kidney_jan10 Also known as: metanephric Bowman's capsule cell fate commitment Definition: The process in which the developmental fate of a cell becomes restricted such that it will develop into a metanephric glomerular parietal epithelial cell. Metanephric glomerular parietal epithelial cells are specialized epithelial cells that form tight junctions as a barrier to protein transport. These cells may also give rise to podocytes.